{
  "gene": "UniProtKB:P30405",
  "term_id": "GO:0005737",
  "gene_name": "Peptidyl-prolyl cis-trans isomerase F, mitochondrial",
  "term_label": "cytoplasm",
  "gene_symbol": "PPIF"
}